{
  "term_label": "vesicle-mediated transport",
  "gene_symbol": "SYT11",
  "gene_name": "Synaptotagmin-11",
  "term_id": "GO:0016192",
  "gene": "UniProtKB:Q9BT88"
}